beta-amylase activity [GO:0016161] (molecular function) References: PMID:18390594 Definition: Catalysis of the reaction: (1,4-alpha-D-glucosyl)(n+1) + H2O = (1,4-alpha-D-glucosyl)(n-1) + alpha-maltose. This reaction is the hydrolysis of 1,4-alpha-glucosidic linkages in polysaccharides so as to remove successive maltose units from the non-reducing ends of the chains. Also known as: glycogenase activity, 4-alpha-D-glucan maltohydrolase activity, beta amylase activity, saccharogen amylase activity Relationships: is a type of amylase activity [GO:0016160]